galactosylceramide metabolic process [GO:0006681] (biological process) Also known as: galactosylceramide metabolism Subtypes: galactosylceramide biosynthetic process [GO:0006682], galactosylceramide catabolic process [GO:0006683] Relationships: is a type of glycosylceramide metabolic process [GO:0006677]; is a type of galactolipid metabolic process [GO:0019374] Sources: GOC:ai Definition: The chemical reactions and pathways involving galactosylceramides, any compound formed by the replacement of the glycosidic hydroxyl group of a cyclic form of galactose by a ceramide group.